cellular response to bile acid [GO:1903413] (biological process) References: PMID:21757002 Sources: GOC:BHF, GOC:TermGenie, GOC:rl, GO_REF:0000071 Relationships: is a type of GO:0071396; is a type of GO:1901701; is a type of response to bile acid [GO:1903412] Definition: Any process that results in a change in state or activity of a cell (in terms of movement, secretion, enzyme production, gene expression, etc.) as a result of a bile acid stimulus.